{
  "term_id": "UNKNOWN:0001",
  "gene_name": "Protein BUD31 homolog",
  "term_label": "Unknown molecular function",
  "gene": "UniProtKB:P41223",
  "gene_symbol": "BUD31"
}